{
  "gene": "UniProtKB:P12525",
  "gene_name": "Putative myc-like protein MYCLP1",
  "gene_symbol": "MYCLP1",
  "term_id": "GO:0006357",
  "term_label": "regulation of transcription by RNA polymerase II"
}